{
  "term_label": "Unknown molecular function",
  "gene_name": "T cell receptor gamma variable 4",
  "term_id": "UNKNOWN:0001",
  "gene_symbol": "TRGV4",
  "gene": "UniProtKB:A0A0C4DH28"
}